{
  "term_id": "UNKNOWN:0002",
  "gene_name": "Zinc finger protein 526",
  "gene": "UniProtKB:Q8TF50",
  "gene_symbol": "ZNF526",
  "term_label": "Unknown biological process"
}